L-alanine biosynthetic process from pyruvate [GO:0019272] (biological process) Also known as: L-alanine anabolism from pyruvate, L-alanine formation from pyruvate, L-alanine synthesis from pyruvate Relationships: is a type of GO:0006090; is a type of L-alanine biosynthetic process [GO:0042852] Sources: GOC:go_curators Definition: The chemical reactions and pathways resulting in the formation of alanine from other compounds, including pyruvate.